{
  "term_label": "protein phosphatase type 2A complex",
  "gene_name": "Serine_threonine-protein phosphatase 2A 55 kDa regulatory subunit B alpha isoform",
  "term_id": "GO:0000159",
  "gene_symbol": "PPP2R2A",
  "gene": "UniProtKB:P63151"
}